{
  "term_label": "bicellular tight junction",
  "gene": "UniProtKB:P78369",
  "term_id": "GO:0005923",
  "gene_name": "Claudin-10",
  "gene_symbol": "CLDN10"
}